{
  "gene_symbol": "DHX40",
  "gene": "UniProtKB:Q8IX18",
  "term_id": "GO:0005681",
  "gene_name": "Probable ATP-dependent RNA helicase DHX40",
  "term_label": "spliceosomal complex"
}